{
  "gene_symbol": "PLA2G4A",
  "gene_name": "Cytosolic phospholipase A2",
  "term_label": "calcium-dependent phospholipase A2 activity",
  "term_id": "GO:0047498",
  "gene": "UniProtKB:P47712"
}